carboxylic acid catabolic process [GO:0046395] (biological process) Relationships: is a type of organic acid catabolic process [GO:0016054]; is a type of carboxylic acid metabolic process [GO:0019752] Definition: The chemical reactions and pathways resulting in the breakdown of carboxylic acids, any organic acid containing one or more carboxyl (-COOH) groups. Subtypes: sulfur amino acid catabolic process [GO:0000098], aromatic amino acid family catabolic process [GO:0009074], GO:0009083, GO:0009091, N-acetylneuraminate catabolic process [GO:0019262], GO:0019501, L-ascorbic acid catabolic process [GO:0019854], leukotriene catabolic process [GO:0036100], alginic acid catabolic process [GO:0042122], chrysobactin catabolic process [GO:0042859], achromobactin catabolic process [GO:0042862], GO:0042865, GO:0043649, gibberellin catabolic process [GO:0045487], phthalate catabolic process [GO:0046239], monocarboxylic acid catabolic process [GO:0072329], GO:0072352, N-acetylmuramic acid catabolic process [GO:0097173], GO:0170040, non-proteinogenic amino acid catabolic process [GO:0170044], fumonisin catabolic process [GO:1900540], gerfelin catabolic process [GO:1900577], endocrocin catabolic process [GO:1900601], tensidol B catabolic process [GO:1900607], GO:1900801, helvolic acid catabolic process [GO:1900811], monodictyphenone catabolic process [GO:1900814], cephalosporin C catabolic process [GO:1901267], fructoselysine catabolic process [GO:1901281], alpha-amino acid catabolic process [GO:1901606], monensin A catabolic process [GO:1901729] Also known as: carboxylic acid breakdown, carboxylic acid catabolism, carboxylic acid degradation Sources: ISBN:0198506732